neurotransmitter receptor transport to plasma membrane [GO:0098877] (biological process) Subtypes: GO:0098969, GO:0099639 Relationships: is a type of protein localization to membrane [GO:0072657]; is a type of GO:0090150; is a type of vesicle-mediated transport to the plasma membrane [GO:0098876]; is a type of neurotransmitter receptor transport [GO:0099637]; is a type of GO:1990778 Definition: The directed movement of neurotransmitter receptor to the plasma membrane in transport vesicles. Sources: GOC:dos